{
  "gene_name": "Uncharacterized protein C17orf80",
  "term_id": "UNKNOWN:0002",
  "term_label": "Unknown biological process",
  "gene": "UniProtKB:Q9BSJ5",
  "gene_symbol": "C17orf80"
}